{
  "gene_symbol": "ITGAL",
  "gene": "UniProtKB:P20701",
  "gene_name": "Integrin alpha-L",
  "term_id": "GO:0007229",
  "term_label": "integrin-mediated signaling pathway"
}